phthalate binding [GO:0035273] (molecular function) Relationships: is a type of carboxylic acid binding [GO:0031406] Definition: Binding to a phthalate, any ester or salt of phthalic acid. References: PMID:31116073